generative cell differentiation [GO:0022619] (biological process) Relationships: is a type of GO:0030154; is part of microgametogenesis [GO:0055046] Sources: GOC:isa_complete Definition: The process in which a relatively unspecialized cell acquires specialized features of a generative cell. The generative cell gives rise to the sperm cells in the male gametophyte.